{
  "term_label": "Unknown cellular component",
  "gene_symbol": "IKBIP",
  "term_id": "UNKNOWN:0003",
  "gene": "UniProtKB:Q70UQ0",
  "gene_name": "Inhibitor of nuclear factor kappa-B kinase-interacting protein"
}